{
  "gene": "UniProtKB:O75352",
  "term_id": "UNKNOWN:0003",
  "term_label": "Unknown cellular component",
  "gene_symbol": "MPDU1",
  "gene_name": "Mannose-P-dolichol utilization defect 1 protein"
}